{
  "gene": "UniProtKB:P78324",
  "term_label": "positive regulation of phagocytosis",
  "gene_symbol": "SIRPA",
  "gene_name": "Tyrosine-protein phosphatase non-receptor type substrate 1",
  "term_id": "GO:0050766"
}